{
  "gene_name": "NADH-ubiquinone oxidoreductase 75 kDa subunit, mitochondrial",
  "term_id": "GO:0008137",
  "term_label": "NADH dehydrogenase (ubiquinone) activity",
  "gene_symbol": "NDUFS1",
  "gene": "UniProtKB:P28331"
}